{
  "term_id": "GO:0005794",
  "term_label": "Golgi apparatus",
  "gene_name": "NEDD4 family-interacting protein 1",
  "gene": "UniProtKB:Q9BT67",
  "gene_symbol": "NDFIP1"
}